{
  "gene_symbol": "HNRNPDL",
  "term_id": "GO:0000785",
  "gene": "UniProtKB:O14979",
  "gene_name": "Heterogeneous nuclear ribonucleoprotein D-like",
  "term_label": "chromatin"
}